G1 to G0 transition [GO:0070314] (biological process) Also known as: G1/G0 transition, establishment of cell quiescence, cell cycle quiescence, stationary phase Regulation: regulated by GO:1903450; negatively regulated by negative regulation of G1 to G0 transition [GO:1903451]; positively regulated by positive regulation of G1 to G0 transition [GO:1903452] Relationships: is a type of cell cycle process [GO:0022402] Subtypes: GO:0070315 Sources: GOC:mah, GOC:mtg_cell_cycle, ISBN:0815316194 Definition: A cell cycle arrest process that results in arrest during G1 phase, whereupon the cell enters a specialized resting state known as G0 or quiescence.